{
  "gene_name": "Adenylate cyclase type 5",
  "term_label": "adenylate cyclase-activating G protein-coupled receptor signaling pathway",
  "term_id": "GO:0007189",
  "gene_symbol": "ADCY5",
  "gene": "UniProtKB:O95622"
}